negative regulation of L-threonine import across plasma membrane [GO:1900927] (biological process) Definition: Any process that stops, prevents or reduces the frequency, rate or extent of L-threonine import into cell. Sources: GOC:TermGenie Also known as: down regulation of L-threonine import, down-regulation of L-threonine import, downregulation of L-threonine import, inhibition of L-threonine import, inhibition of L-threonine uptake, down regulation of L-threonine uptake, down-regulation of L-threonine uptake, downregulation of L-threonine uptake, negative regulation of L-threonine uptake Relationships: is_a negative regulation of organic acid transport [GO:0032891]; is_a negative regulation of transmembrane transport [GO:0034763]; is a type of GO:0051956; is a type of regulation of L-threonine import across plasma membrane [GO:1900926]; negatively regulates L-threonine import across plasma membrane [GO:1903807]